{
  "term_id": "GO:0005102",
  "term_label": "signaling receptor binding",
  "gene_name": "Putative HLA class I histocompatibility antigen, alpha chain H",
  "gene": "UniProtKB:P01893",
  "gene_symbol": "HLA-H"
}